{
  "term_label": "RNA polymerase II cis-regulatory region sequence-specific DNA binding",
  "gene_symbol": "SOX8",
  "gene_name": "Transcription factor SOX-8",
  "term_id": "GO:0000978",
  "gene": "UniProtKB:P57073"
}